4-nitrocatechol 4-monooxygenase activity [GO:0018592] (molecular function) Definition: Catalysis of the reaction: 4-nitrocatechol + NAD(P)H + O2 = 2-hydroxy-1,4-benzoquinone + nitrite + NAD(P)+ + H2O. Relationships: is_a oxidoreductase activity, acting on paired donors, with incorporation or reduction of molecular oxygen, NAD(P)H as one donor, and incorporation of one atom of oxygen [GO:0016709] Sources: EC:1.14.13.166